{
  "term_id": "GO:0005737",
  "gene": "UniProtKB:P61981",
  "term_label": "cytoplasm",
  "gene_name": "14-3-3 protein gamma",
  "gene_symbol": "YWHAG"
}